{
  "gene_symbol": "ZNF512B",
  "gene": "UniProtKB:Q96KM6",
  "gene_name": "Zinc finger protein 512B",
  "term_id": "UNKNOWN:0001",
  "term_label": "Unknown molecular function"
}